{
  "term_label": "DNA-binding transcription factor activity, RNA polymerase II-specific",
  "gene": "UniProtKB:Q9HD90",
  "term_id": "GO:0000981",
  "gene_symbol": "NEUROD4",
  "gene_name": "Neurogenic differentiation factor 4"
}